acridone synthase activity [GO:0050635] (molecular function) Sources: EC:2.3.1.159, RHEA:22224 Also known as: malonyl-CoA:N-methylanthraniloyl-CoA malonyltransferase (cyclizing) Definition: Catalysis of the reaction: N-methylanthranilyl-CoA + 3 H+ + 3 malonyl-CoA = 1,3-dihydroxy-N-methylacridone + 3 CO2 + 4 CoA + H2O. Relationships: is a type of acyltransferase activity, transferring groups other than amino-acyl groups [GO:0016747]